{
  "gene_name": "Olfactory receptor 4C16",
  "gene_symbol": "OR4C16",
  "gene": "UniProtKB:Q8NGL9",
  "term_id": "GO:0005886",
  "term_label": "plasma membrane"
}